{
  "gene_name": "Glycosyltransferase-like domain-containing protein 1",
  "gene": "UniProtKB:Q4AE62",
  "term_id": "GO:0005634",
  "term_label": "nucleus",
  "gene_symbol": "GTDC1"
}